{
  "gene_symbol": "TNNT2",
  "term_id": "GO:0005861",
  "gene": "UniProtKB:P45379",
  "term_label": "troponin complex",
  "gene_name": "Troponin T, cardiac muscle"
}